{
  "gene_name": "Coiled-coil domain containing 92B",
  "term_id": "UNKNOWN:0002",
  "gene_symbol": "CCDC92B",
  "term_label": "Unknown biological process",
  "gene": "UniProtKB:A0A8I5KY20"
}